{
  "gene_name": "V-type proton ATPase 116 kDa subunit a 1",
  "term_id": "GO:0005886",
  "gene": "UniProtKB:Q93050",
  "gene_symbol": "ATP6V0A1",
  "term_label": "plasma membrane"
}